{
  "term_id": "UNKNOWN:0001",
  "gene_symbol": "CHI3L2",
  "gene": "UniProtKB:Q15782",
  "term_label": "Unknown molecular function",
  "gene_name": "Chitinase-3-like protein 2"
}